{
  "term_label": "nucleus",
  "term_id": "GO:0005634",
  "gene": "UniProtKB:Q13106",
  "gene_symbol": "ZNF154",
  "gene_name": "Zinc finger protein 154"
}